lignostilbene alpha beta-dioxygenase activity [GO:0050054] (molecular function) Sources: EC:1.13.11.43, RHEA:21340 Also known as: lignostilbene ab-dioxygenase activity, 1,2-bis(4-hydroxy-3-methoxyphenyl)ethylene:oxygen oxidoreductase (alphabeta-bond-cleaving), lignostilbene alphabeta-dioxygenase activity Definition: Catalysis of the reaction: 1,2-bis(4-hydroxy-3-methoxyphenyl)ethylene + O2 = 2 vanillin. Relationships: is a type of oxidoreductase activity, acting on single donors with incorporation of molecular oxygen, incorporation of two atoms of oxygen [GO:0016702]